{
  "term_id": "GO:0003735",
  "gene": "UniProtKB:P82933",
  "gene_symbol": "MRPS9",
  "gene_name": "Small ribosomal subunit protein uS9m",
  "term_label": "structural constituent of ribosome"
}